{
  "term_label": "P granule",
  "gene": "UniProtKB:Q9HCE1",
  "gene_symbol": "MOV10",
  "term_id": "GO:0043186",
  "gene_name": "Helicase MOV-10"
}